{
  "term_label": "syntaxin binding",
  "gene": "UniProtKB:Q9BV40",
  "gene_symbol": "VAMP8",
  "gene_name": "Vesicle-associated membrane protein 8",
  "term_id": "GO:0019905"
}